{
  "term_id": "GO:0016477",
  "gene": "UniProtKB:Q9BX67",
  "gene_symbol": "JAM3",
  "gene_name": "Junctional adhesion molecule C",
  "term_label": "cell migration"
}